melatonin metabolic process [GO:0030186] (biological process) Also known as: melatonin metabolism Subtypes: melatonin biosynthetic process [GO:0030187], melatonin catabolic process [GO:0042442] Sources: GOC:mah, ISBN:0198506732 Relationships: is a type of indole-containing compound metabolic process [GO:0042430]; is a type of hormone metabolic process [GO:0042445]; is a type of GO:0043603 Definition: The chemical reactions and pathways involving melatonin (N-acetyl-5-methoxytryptamine).